{
  "term_id": "UNKNOWN:0002",
  "term_label": "Unknown biological process",
  "gene_name": "Putative uncharacterized protein encoded by LINC00208",
  "gene": "UniProtKB:Q96KT6",
  "gene_symbol": "LINC00208"
}